{
  "gene_symbol": "SPRYD3",
  "gene": "UniProtKB:Q8NCJ5",
  "gene_name": "SPRY domain-containing protein 3",
  "term_label": "protein-macromolecule adaptor activity",
  "term_id": "GO:0030674"
}